thick ascending limb development [GO:0072023] (biological process) Subtypes: metanephric thick ascending limb development [GO:0072233] Sources: GOC:mtg_kidney_jan10 Relationships: is a type of nephron tubule development [GO:0072080]; is part of distal tubule development [GO:0072017] Also known as: TAL development Definition: The process whose specific outcome is the progression of the thick ascending limb over time, from its formation to the mature structure. The thick ascending limb is the last part of the loop of Henle. Its thick, mitochondria-rich epithelium characterizes the outer medulla, and is responsible for very avid active salt transport. At the macula densa, the thick ascending limb connects to the distal convoluted tubule.